negative regulation of synaptic metaplasticity [GO:0031917] (biological process) Relationships: is a type of negative regulation of synaptic plasticity [GO:0031914]; is a type of regulation of synaptic metaplasticity [GO:0031916] Definition: A process that decreases synaptic metaplasticity. Metaplasticity is a higher-order form of plasticity and is manifest as a change in the ability to induce subsequent synaptic plasticity that is the ability of synapses to change as circumstances require. References: PMID:8658594 Sources: GOC:mah Also known as: down regulation of synaptic metaplasticity, down-regulation of synaptic metaplasticity, downregulation of synaptic metaplasticity, inhibition of synaptic metaplasticity